{
  "gene_symbol": "NANOG",
  "term_label": "RNA polymerase II cis-regulatory region sequence-specific DNA binding",
  "gene": "UniProtKB:Q9H9S0",
  "term_id": "GO:0000978",
  "gene_name": "Homeobox protein NANOG"
}